regulation of autophagy of mitochondrion [GO:1903146] (biological process) Definition: Any process that modulates the frequency, rate or extent of mitochondrion degradation by an autophagic process. Subtypes: regulation of mitophagy [GO:1901524], negative regulation of autophagy of mitochondrion [GO:1903147], positive regulation of autophagy of mitochondrion [GO:1903599] Relationships: is a type of regulation of autophagy [GO:0010506]; RO_0002211 autophagy of mitochondrion [GO:0000422] Also known as: regulation of mitochondrion degradation References: PMID:24600391 Sources: GOC:PARL, GOC:TermGenie, GOC:autophagy, GOC:bf, GO_REF:0000058